beta-glucan biosynthetic process [GO:0051274] (biological process) Regulation: regulated by GO:0032951 Relationships: is a type of glucan biosynthetic process [GO:0009250]; is a type of beta-glucan metabolic process [GO:0051273] Subtypes: (1->3)-beta-D-glucan biosynthetic process [GO:0006075], GO:0006078, GO:0030244, cell wall beta-glucan biosynthetic process [GO:0034410] Sources: GOC:ai Definition: The chemical reactions and pathways resulting in the formation of beta-glucans. Also known as: beta-glucan anabolism, beta-glucan biosynthesis, beta-glucan formation, beta-glucan synthesis